L-fucose catabolic process [GO:0042355] (biological process) Sources: GOC:jl Also known as: L-fucose breakdown, L-fucose catabolism, L-fucose degradation Relationships: is_a fucose catabolic process [GO:0019317]; is a type of L-fucose metabolic process [GO:0042354] Definition: The chemical reactions and pathways resulting in the breakdown of L-fucose (6-deoxy-Lgalactose).